tartrate biosynthetic process [GO:1901277] (biological process) Also known as: tartrate anabolism, tartrate biosynthesis, tartrate formation, tartrate synthesis Relationships: is a type of biosynthetic process [GO:0009058]; is a type of GO:1901275 Sources: GOC:TermGenie, GOC:yaf, UniPathway:UPA00839 Definition: The chemical reactions and pathways resulting in the formation of tartrate.